{
  "gene": "UniProtKB:A6NC57",
  "term_id": "UNKNOWN:0002",
  "gene_symbol": "ANKRD62",
  "gene_name": "Ankyrin repeat domain-containing protein 62",
  "term_label": "Unknown biological process"
}